{
  "term_id": "GO:0016020",
  "gene": "UniProtKB:Q8WUJ1",
  "gene_symbol": "CYB5D2",
  "gene_name": "Neuferricin",
  "term_label": "membrane"
}